late distal convoluted tubule development [GO:0072068] (biological process) Relationships: is a type of GO:0072009; is part of distal convoluted tubule development [GO:0072025] Definition: The process whose specific outcome is the progression of the late distal convoluted tubule over time, from its formation to the mature structure. The late distal convoluted tubule contains DCT cells and intercalated (IC) alpha and beta cells and is vasopressin-sensitive. Sources: GOC:mtg_kidney_jan10 Subtypes: metanephric late distal convoluted tubule development [GO:0072225]